{
  "gene_symbol": "LCMT2",
  "term_label": "tRNA methylation",
  "gene": "UniProtKB:O60294",
  "gene_name": "tRNA wybutosine-synthesizing protein 4",
  "term_id": "GO:0030488"
}